ventral midline determination [GO:0007371] (biological process) Also known as: determination of anterior border of ventral midline, determination of posterior border of ventral midline Relationships: is_a regionalization [GO:0003002]; is part of GO:0007418 Definition: The regionalization process in which the area where the ventral midline will form is specified. Sources: GOC:bf, GOC:isa_complete, GOC:vk